Wnt-Frizzled-LRP5/6 complex [GO:1990851] (cellular component) Definition: A protein complex containing a secreted Wnt protein associated with its receptor, Frizzled (Fz), and co-receptor low density lipoprotein receptor-related protein 5 (LRP5) or LRP6. Relationships: is a type of GO:0098797 Note: Given the number of Wnt proteins, Frizzled proteins and LRP proteins, many different trimeric complexes are likely to form. Also known as: Wnt receptor complex, Wnt-FZD-LRP5/6 trimeric complex, Wnt.Fz.LRP ternary complex, Fz/Wnt/LRP6 complex, WNT-FZD-LRP5 complex, WNT-FZD-LRP6 complex, Frizzled-LRP5/6 complex, Wnt-induced Frizzled-LRP5/6 complex References: PMID:11448771, PMID:20093360 Sources: GOC:PARL, GOC:bf